{
  "term_id": "GO:0003823",
  "gene_name": "Immunoglobulin heavy variable 4-30-4",
  "term_label": "antigen binding",
  "gene_symbol": "IGHV4-30-4",
  "gene": "UniProtKB:P0DP06"
}